{
  "term_label": "calmodulin binding",
  "gene_symbol": "SPA17",
  "gene": "UniProtKB:Q15506",
  "term_id": "GO:0005516",
  "gene_name": "Sperm surface protein Sp17"
}